MHC class II receptor activity [GO:0032395] (molecular function) Note: Note that this term is intended for annotation of gene products that act as receptors for MHC class II protein complexes, not for components of the MHC class II protein complexes themselves. Relationships: is a type of transmembrane signaling receptor activity [GO:0004888]; is a type of GO:0140375; has part GO:0042289 Also known as: T cell receptor activity, alpha-beta T cell receptor activity, gamma-delta T cell receptor activity Definition: Combining with an MHC class II protein complex and transmitting the signal from one side of the membrane to the other to initiate a change in cell activity. Sources: GOC:add, GOC:signaling, ISBN:0781735149